ADPG pyrophosphorylase complex [GO:0030929] (cellular component) Definition: Complex that possesses ADPG pyrophosphorylase activity. In all organisms where it has been found, the complex is a tetramer. In bacteria, it is a homotetramer. In plants, the complex is a heterotetramer composed small and large subunits. Subtypes: homotetrameric ADPG pyrophosphorylase complex [GO:0030930], heterotetrameric ADPG pyrophosphorylase complex [GO:0030931] References: PMID:9680965 Sources: GOC:tb Relationships: is a type of intracellular protein-containing complex [GO:0140535]; is a type of catalytic complex [GO:1902494]